response to diterpene [GO:1904629] (biological process) Relationships: is a type of response to lipid [GO:0033993] References: PMID:19765580 Sources: GOC:TermGenie, GO_REF:0000071 Definition: Any process that results in a change in state or activity of a cell or an organism (in terms of movement, secretion, enzyme production, gene expression, etc.) as a result of a diterpene stimulus. Subtypes: GO:1904630